ADP-thymidine kinase activity [GO:0047628] (molecular function) Definition: Catalysis of the reaction: ADP + thymidine = AMP + thymidine 5'-phosphate. Relationships: is a type of kinase activity [GO:0016301]; is a type of phosphotransferase activity, alcohol group as acceptor [GO:0016773] Sources: EC:2.7.1.118, MetaCyc:ADP--THYMIDINE-KINASE-RXN Also known as: ADP:dThd phosphotransferase activity, ADP:thymidine 5'-phosphotransferase activity, adenosine diphosphate-thymidine phosphotransferase activity